membrane fusion involved in viral entry into host cell [GO:0039663] (BP) Definition: Merging of the virion membrane and a host membrane (host plasma membrane or host organelle membrane) that is involved in the uptake of a virus into a host cell. Sources: GOC:bf, GOC:jl, UniProtKB-KW:KW-1168 Relationships: is a type of viral process [GO:0016032] Subtypes: fusion of virus membrane with host plasma membrane [GO:0019064], fusion of virus membrane with host endosome membrane [GO:0039654] Also known as: fusion of virus membrane with host membrane, fusion of virus membrane with host membrane during viral entry, viral entry into host cell via membrane fusion